{
  "term_id": "UNKNOWN:0003",
  "gene": "UniProtKB:Q86XK2",
  "gene_name": "F-box only protein 11",
  "gene_symbol": "FBXO11",
  "term_label": "Unknown cellular component"
}